{
  "term_label": "sperm head",
  "gene": "UniProtKB:Q9H112",
  "gene_name": "Cystatin-11",
  "term_id": "GO:0061827",
  "gene_symbol": "CST11"
}